{
  "gene_symbol": "ZNF485",
  "gene": "UniProtKB:Q8NCK3",
  "term_id": "GO:0006357",
  "gene_name": "Zinc finger protein 485",
  "term_label": "regulation of transcription by RNA polymerase II"
}